heme a catabolic process [GO:0046161] (BP) Definition: The chemical reactions and pathways resulting in the breakdown of heme a, a derivative of heme found in cytochrome aa3. Also known as: haem a catabolic process, haem a catabolism, heme a breakdown, heme a catabolism, heme a degradation References: PMID:28352909 Sources: GOC:curators Relationships: is a type of heme catabolic process [GO:0042167]